karyomere assembly [GO:0061471] (biological process) Relationships: is a type of organelle assembly [GO:0070925]; is_a mitotic cell cycle process [GO:1903047]; BFO_0000050 mitotic nuclear membrane reassembly [GO:0007084] Definition: The process where the nuclear membrane engulfs condensed chromosomes to form karyomeres during M phase of the mitotic cell cycle. References: PMID:9732278 Sources: GOC:dph